thiamine diphosphokinase activity [GO:0004788] (molecular function) Sources: RHEA:11576 Definition: Catalysis of the reaction: ATP + thiamine = AMP + thiamine diphosphate. Also known as: thiamin diphosphokinase activity, thiamin pyrophosphokinase activity, thiamine pyrophosphokinase activity, ATP:thiamin pyrophosphotransferase activity, ATP:thiamine diphosphotransferase activity, TPTase activity, thiamin pyrophosphotransferase activity, thiamin:ATP pyrophosphotransferase activity, thiaminokinase activity Relationships: is a type of diphosphotransferase activity [GO:0016778]